{
  "gene_symbol": "OLIG3",
  "gene": "UniProtKB:Q7RTU3",
  "gene_name": "Oligodendrocyte transcription factor 3",
  "term_label": "nucleus",
  "term_id": "GO:0005634"
}